{
  "term_id": "UNKNOWN:0003",
  "term_label": "Unknown cellular component",
  "gene": "UniProtKB:P61601",
  "gene_name": "Neurocalcin-delta",
  "gene_symbol": "NCALD"
}